auxin metabolic process [GO:0009850] (biological process) Sources: GOC:lr Relationships: is a type of GO:0042445 Definition: The chemical reactions and pathways involving auxins, a group of plant hormones that regulate aspects of plant growth. Regulation: regulated by regulation of auxin metabolic process [GO:0090354]; positively regulated by positive regulation of auxin metabolic process [GO:0090355]; negatively regulated by GO:0090356 Also known as: auxin metabolism Subtypes: GO:0009851, auxin catabolic process [GO:0009852], auxin conjugate metabolic process [GO:0010249], indolebutyric acid metabolic process [GO:0080024]